{
  "gene_name": "Phospholipase ABHD3",
  "gene": "UniProtKB:Q8WU67",
  "gene_symbol": "ABHD3",
  "term_id": "UNKNOWN:0003",
  "term_label": "Unknown cellular component"
}